autosome [GO:0030849] (cellular component) Relationships: is a type of chromosome [GO:0005694] Note: Note that this term is mainly relevant in organisms that have both sex chromosomes and non-sex-determining chromosomes in an individual organism. Sources: GOC:mah Definition: Any chromosome other than a sex chromosome.